{
  "gene_name": "Transcriptional enhancer factor TEF-5",
  "term_id": "GO:0006357",
  "gene": "UniProtKB:Q99594",
  "gene_symbol": "TEAD3",
  "term_label": "regulation of transcription by RNA polymerase II"
}